{
  "term_id": "UNKNOWN:0002",
  "term_label": "Unknown biological process",
  "gene_symbol": "ZNF839",
  "gene_name": "Zinc finger protein 839",
  "gene": "UniProtKB:A8K0R7"
}